{
  "term_label": "regulation of transcription by RNA polymerase II",
  "gene": "UniProtKB:Q04741",
  "gene_name": "Homeobox protein EMX1",
  "term_id": "GO:0006357",
  "gene_symbol": "EMX1"
}